{
  "gene_name": "Proline-rich transmembrane protein 1",
  "term_label": "signaling receptor regulator activity",
  "term_id": "GO:0030545",
  "gene_symbol": "PRRT1",
  "gene": "UniProtKB:Q99946"
}